actomyosin contractile ring actin filament [GO:1903144] (cellular component) References: PMID:20807799, PMID:24954052 Sources: GOC:TermGenie, GO_REF:0000064 Definition: Any actin filament that is part of a actomyosin contractile ring. Relationships: is a type of actin filament [GO:0005884]; is part of actomyosin contractile ring [GO:0005826] Also known as: actin filament of CAR, actin filament of actomyosin contractile ring, actin filament of actomyosin ring, actin filament of contractile actomyosin ring, actin filament of cytokinetic ring